{
  "term_id": "GO:0030335",
  "term_label": "positive regulation of cell migration",
  "gene_symbol": "CX3CL1",
  "gene": "UniProtKB:P78423",
  "gene_name": "Fractalkine"
}